{
  "term_id": "GO:0005739",
  "gene_name": "Transmembrane protein 223",
  "gene_symbol": "TMEM223",
  "gene": "UniProtKB:A0PJW6",
  "term_label": "mitochondrion"
}